{
  "term_id": "GO:0005198",
  "gene_name": "Uroplakin-1b",
  "gene": "UniProtKB:O75841",
  "term_label": "structural molecule activity",
  "gene_symbol": "UPK1B"
}